{
  "gene_symbol": "IL21R",
  "gene_name": "Interleukin-21 receptor",
  "term_id": "GO:0009897",
  "gene": "UniProtKB:Q9HBE5",
  "term_label": "external side of plasma membrane"
}